regulation of T cell tolerance induction [GO:0002664] (biological process) Sources: GOC:add Also known as: regulation of T lymphocyte tolerance induction, regulation of T-cell tolerance induction, regulation of T-lymphocyte tolerance induction Relationships: is a type of GO:0002643; regulates T cell tolerance induction [GO:0002517] Definition: Any process that modulates the frequency, rate, or extent of T cell tolerance induction. Subtypes: negative regulation of T cell tolerance induction [GO:0002665], GO:0002666, regulation of T cell anergy [GO:0002667], GO:0002849